clypeus development [GO:0048723] (biological process) Relationships: is a type of anatomical structure development [GO:0048856]; is part of clypeo-labral disc development [GO:0035213] Sources: GOC:rc Definition: The process whose specific outcome is the progression of the clypeus over time, from its formation to the mature structure. The clypeus is the shield-shaped plate on an insect's head.